{
  "term_label": "cytoplasm",
  "gene_name": "Ferritin heavy polypeptide-like 17",
  "term_id": "GO:0005737",
  "gene_symbol": "FTHL17",
  "gene": "UniProtKB:Q9BXU8"
}